{
  "term_id": "GO:0005615",
  "gene_symbol": "WNT5A",
  "term_label": "extracellular space",
  "gene": "UniProtKB:P41221",
  "gene_name": "Protein Wnt-5a"
}